{
  "gene_name": "Progestin and adipoQ receptor family member 3",
  "gene_symbol": "PAQR3",
  "term_label": "protein localization to Golgi apparatus",
  "gene": "UniProtKB:Q6TCH7",
  "term_id": "GO:0034067"
}